{
  "gene_symbol": "TRAF3IP1",
  "term_label": "ciliary basal body",
  "gene": "UniProtKB:Q8TDR0",
  "gene_name": "TRAF3-interacting protein 1",
  "term_id": "GO:0036064"
}